{
  "gene_name": "NHL-repeat-containing protein 4",
  "term_label": "Unknown biological process",
  "gene_symbol": "NHLRC4",
  "term_id": "UNKNOWN:0002",
  "gene": "UniProtKB:P0CG21"
}